{
  "term_label": "Unknown molecular function",
  "gene_name": "Neuronal membrane glycoprotein M6-a",
  "gene_symbol": "GPM6A",
  "term_id": "UNKNOWN:0001",
  "gene": "UniProtKB:P51674"
}